{
  "gene": "UniProtKB:P56470",
  "term_id": "UNKNOWN:0002",
  "gene_name": "Galectin-4",
  "gene_symbol": "LGALS4",
  "term_label": "Unknown biological process"
}